{
  "term_id": "GO:0003924",
  "term_label": "GTPase activity",
  "gene_name": "Guanine nucleotide-binding protein G(t) subunit alpha-3",
  "gene": "UniProtKB:A8MTJ3",
  "gene_symbol": "GNAT3"
}